{
  "gene": "UniProtKB:P46934",
  "gene_symbol": "NEDD4",
  "term_id": "GO:0061630",
  "term_label": "ubiquitin protein ligase activity",
  "gene_name": "E3 ubiquitin-protein ligase NEDD4"
}